{
  "gene_symbol": "GNG3",
  "gene": "UniProtKB:P63215",
  "gene_name": "Guanine nucleotide-binding protein G(I)_G(S)_G(O) subunit gamma-3",
  "term_label": "G-protein beta-subunit binding",
  "term_id": "GO:0031681"
}